pyrimidine deoxyribonucleotide metabolic process [GO:0009219] (biological process) Sources: GOC:go_curators, ISBN:0198506732 Relationships: is a type of pyrimidine nucleotide metabolic process [GO:0006220]; is a type of GO:0009394 Also known as: pyrimidine deoxyribonucleotide metabolism Subtypes: pyrimidine deoxyribonucleotide biosynthetic process [GO:0009221], pyrimidine deoxyribonucleotide catabolic process [GO:0009223], pyrimidine deoxyribonucleotide interconversion [GO:0015955], dCDP metabolic process [GO:0046062], dCMP metabolic process [GO:0046063], dCTP metabolic process [GO:0046065], dTDP metabolic process [GO:0046072], dTMP metabolic process [GO:0046073], dTTP metabolic process [GO:0046075], dUDP metabolic process [GO:0046077], dUMP metabolic process [GO:0046078], dUTP metabolic process [GO:0046080] Definition: The chemical reactions and pathways involving a pyrimidine deoxynucleotide, a compound consisting of nucleoside (a pyrimidine base linked to a deoxyribose sugar) esterified with a phosphate group at either the 3' or 5'-hydroxyl group of the sugar.